{
  "term_id": "UNKNOWN:0003",
  "gene_symbol": "NCR3",
  "gene_name": "Natural cytotoxicity triggering receptor 3",
  "gene": "UniProtKB:O14931",
  "term_label": "Unknown cellular component"
}